{
  "gene": "UniProtKB:A6NDV4",
  "gene_name": "Transmembrane protein 8B",
  "term_label": "Unknown cellular component",
  "gene_symbol": "TMEM8B",
  "term_id": "UNKNOWN:0003"
}